{
  "gene_symbol": "WDR26",
  "term_id": "UNKNOWN:0001",
  "gene_name": "WD repeat-containing protein 26",
  "term_label": "Unknown molecular function",
  "gene": "UniProtKB:Q9H7D7"
}